{
  "gene_symbol": "ATG4D",
  "term_label": "protein-phosphatidylethanolamide deconjugating activity",
  "term_id": "GO:0019786",
  "gene_name": "Cysteine protease ATG4D",
  "gene": "UniProtKB:Q86TL0"
}